{
  "gene_name": "Ankyrin repeat and SOCS box protein 4",
  "gene_symbol": "ASB4",
  "gene": "UniProtKB:Q9Y574",
  "term_label": "Unknown molecular function",
  "term_id": "UNKNOWN:0001"
}